{
  "term_label": "translation activator activity",
  "gene": "UniProtKB:A9UHW6",
  "term_id": "GO:0008494",
  "gene_symbol": "MIF4GD",
  "gene_name": "MIF4G domain-containing protein"
}